seminal clot liquefaction [GO:0070684] (biological process) Definition: The reproductive process in which coagulated semen becomes liquid following ejaculation, allowing the progressive release of motile spermatozoa. Also known as: semen liquefaction References: PMID:18482984 Sources: GOC:mah Relationships: is a type of multicellular organismal reproductive process [GO:0048609]; is part of GO:0007320